{
  "gene": "UniProtKB:Q4LDE5",
  "term_id": "UNKNOWN:0001",
  "gene_symbol": "SVEP1",
  "term_label": "Unknown molecular function",
  "gene_name": "Sushi, von Willebrand factor type A, EGF and pentraxin domain-containing protein 1"
}